{
  "term_label": "structural constituent of ribosome",
  "gene_name": "Small ribosomal subunit protein eS21",
  "gene": "UniProtKB:P63220",
  "gene_symbol": "RPS21",
  "term_id": "GO:0003735"
}